D-lactate dehydrogenase (NAD+) activity [GO:0008720] (molecular function) Also known as: D-lactate dehydrogenase activity, D-lactic acid dehydrogenase activity, D-lactic dehydrogenase activity Sources: RHEA:16369 Definition: Catalysis of the reaction: (R)-lactate + NAD+ = H+ + NADH + pyruvate. Relationships: is a type of D-lactate dehydrogenase activity [GO:0047809]; is a type of (2R)-2-hydroxyacid dehydrogenase (NAD+) activity [GO:0140175]